{
  "term_label": "MHC class II protein complex binding",
  "term_id": "GO:0023026",
  "gene_name": "HLA class II histocompatibility antigen, DM alpha chain",
  "gene_symbol": "HLA-DMA",
  "gene": "UniProtKB:P28067"
}